negative regulation of cardiac muscle hypertrophy in response to stress [GO:1903243] (biological process) References: PMID:19287093 Sources: GOC:BHF, GOC:TermGenie, GOC:rl, GO_REF:0000058 Also known as: down regulation of cardiac muscle hypertrophy in response to stress, down-regulation of cardiac muscle hypertrophy in response to stress, downregulation of cardiac muscle hypertrophy in response to stress, inhibition of cardiac muscle hypertrophy in response to stress Definition: Any process that stops, prevents or reduces the frequency, rate or extent of cardiac muscle hypertrophy in response to stress. Relationships: is a type of negative regulation of cardiac muscle hypertrophy [GO:0010614]; is a type of negative regulation of cardiac muscle adaptation [GO:0010616]; is a type of regulation of cardiac muscle hypertrophy in response to stress [GO:1903242]; negatively regulates GO:0014898